chloroplast targeting sequence binding [GO:0030941] (molecular function) Relationships: is a type of signal sequence binding [GO:0005048] Definition: Binding to a chloroplast targeting sequence, a specific peptide sequence that acts as a signal to localize the protein within the chloroplast. Sources: GOC:mah